{
  "gene": "UniProtKB:P18054",
  "gene_name": "Polyunsaturated fatty acid lipoxygenase ALOX12",
  "gene_symbol": "ALOX12",
  "term_label": "arachidonate 15-lipoxygenase activity",
  "term_id": "GO:0050473"
}